{
  "gene_name": "CAAX box protein 1",
  "gene_symbol": "RTL8C",
  "term_id": "UNKNOWN:0001",
  "gene": "UniProtKB:O15255",
  "term_label": "Unknown molecular function"
}